negative regulation of eating behavior [GO:1903999] (biological process) Subtypes: negative regulation of nematode pharyngeal pumping [GO:1903745] Relationships: is a type of regulation of eating behavior [GO:1903998]; is a type of negative regulation of feeding behavior [GO:2000252]; negatively regulates GO:0042755 References: PMID:11961051 Sources: GOC:TermGenie, GO_REF:0000058 Also known as: down regulation of eating behavior, down regulation of eating behaviour, down-regulation of eating behavior, down-regulation of eating behaviour, downregulation of eating behavior, downregulation of eating behaviour, negative regulation of eating behaviour, inhibition of eating behavior, inhibition of eating behaviour Definition: Any process that stops, prevents or reduces the frequency, rate or extent of eating behavior.